group A colicin transport [GO:0042915] (biological process) Relationships: is a type of colicin transport [GO:0042914] References: PMID:9171417 Sources: GOC:jl Definition: The directed movement of group A colicins (colicins E1, E2, E3, A, K, and N) into, out of or within a cell, or between cells, by means of some agent such as a transporter or pore.